{
  "gene_symbol": "CCDC88A",
  "gene": "UniProtKB:Q3V6T2",
  "term_id": "GO:0030705",
  "term_label": "cytoskeleton-dependent intracellular transport",
  "gene_name": "Girdin"
}